{
  "term_id": "UNKNOWN:0003",
  "gene_symbol": "HECTD1",
  "gene": "UniProtKB:Q9ULT8",
  "term_label": "Unknown cellular component",
  "gene_name": "E3 ubiquitin-protein ligase HECTD1"
}